{
  "gene_name": "Disks large homolog 4",
  "gene_symbol": "DLG4",
  "gene": "UniProtKB:P78352",
  "term_id": "GO:0019901",
  "term_label": "protein kinase binding"
}